{
  "gene_name": "5'-AMP-activated protein kinase subunit gamma-3",
  "gene": "UniProtKB:Q9UGI9",
  "term_id": "GO:0016208",
  "term_label": "AMP binding",
  "gene_symbol": "PRKAG3"
}